tRNA (m1A) methyltransferase complex [GO:0031515] (cellular component) Relationships: is a type of tRNA methyltransferase complex [GO:0043527] Definition: A protein complex involved in the catalysis of the formation of the modified nucleotide 1-methyladenosine (m1A) in tRNA. In yeast, it is a heterotetramer of two subunits, Gcd10p and Gcd14p, while in bacteria and archaea it is a homotetramer. References: PMID:10779558, PMID:14739239